{
  "term_id": "GO:0007219",
  "gene_name": "Probable E3 ubiquitin-protein ligase DTX3",
  "term_label": "Notch signaling pathway",
  "gene": "UniProtKB:Q8N9I9",
  "gene_symbol": "DTX3"
}